{
  "gene": "UniProtKB:O00213",
  "term_id": "GO:0005737",
  "gene_name": "Amyloid beta precursor protein binding family B member 1",
  "gene_symbol": "APBB1",
  "term_label": "cytoplasm"
}